{
  "gene_name": "Neuropilin-1",
  "gene": "UniProtKB:O14786",
  "gene_symbol": "NRP1",
  "term_label": "focal adhesion",
  "term_id": "GO:0005925"
}